positive regulation of chronic inflammatory response to antigenic stimulus [GO:0002876] (biological process) Sources: GOC:add Also known as: up regulation of chronic inflammatory response to antigenic stimulus, up-regulation of chronic inflammatory response to antigenic stimulus, upregulation of chronic inflammatory response to antigenic stimulus, activation of chronic inflammatory response to antigenic stimulus, stimulation of chronic inflammatory response to antigenic stimulus Definition: Any process that activates or increases the frequency, rate, or extent of a chronic inflammatory response to an antigenic stimulus. Relationships: is a type of GO:0002678; is a type of GO:0002863; is a type of regulation of chronic inflammatory response to antigenic stimulus [GO:0002874]; positively regulates GO:0002439